{
  "term_id": "GO:0005634",
  "gene_name": "Zinc finger protein 266",
  "gene": "UniProtKB:Q14584",
  "gene_symbol": "ZNF266",
  "term_label": "nucleus"
}